{
  "gene": "UniProtKB:P15529",
  "term_label": "negative regulation of complement activation, classical pathway",
  "gene_name": "Membrane cofactor protein",
  "term_id": "GO:0045959",
  "gene_symbol": "CD46"
}